{
  "gene_symbol": "EXD1",
  "gene_name": "piRNA biogenesis protein EXD1",
  "term_label": "PET complex",
  "term_id": "GO:1990923",
  "gene": "UniProtKB:Q8NHP7"
}